{
  "gene_symbol": "TEKT5",
  "gene": "UniProtKB:Q96M29",
  "gene_name": "Tektin-5",
  "term_id": "GO:0015630",
  "term_label": "microtubule cytoskeleton"
}